{
  "gene_name": "2',5'-phosphodiesterase 12",
  "gene_symbol": "PDE12",
  "term_id": "GO:0000175",
  "gene": "UniProtKB:Q6L8Q7",
  "term_label": "3'-5'-RNA exonuclease activity"
}